{
  "gene_symbol": "CCL21",
  "term_id": "GO:0048245",
  "gene_name": "C-C motif chemokine 21",
  "gene": "UniProtKB:O00585",
  "term_label": "eosinophil chemotaxis"
}